{
  "term_label": "cytosol",
  "term_id": "GO:0005829",
  "gene_symbol": "CASTOR3P",
  "gene": "UniProtKB:Q8NAP1",
  "gene_name": "Putative protein CASTOR3P"
}